positive regulation of venous endothelial cell fate commitment [GO:2000789] (biological process) Relationships: is a type of positive regulation of cell fate commitment [GO:0010455]; is a type of positive regulation of blood vessel endothelial cell differentiation [GO:0110058]; is a type of GO:2000787; positively regulates venous endothelial cell fate commitment [GO:0060845] References: PMID:11585794 Definition: Any process that activates or increases the frequency, rate or extent of venous endothelial cell fate commitment.